regulation of (R)-mevalonic acid biosynthetic process [GO:0106107] (biological process) References: PMID:24296663 Sources: GOC:BHF, GOC:BHF_miRNA, GOC:rph Subtypes: negative regulation of (R)-mevalonic acid biosynthetic process [GO:0106108], positive regulation of (R)-mevalonic acid biosynthetic process [GO:0106109] Relationships: is a type of GO:0009889; is a type of GO:0062012; regulates (R)-mevalonic acid biosynthetic process [GO:1901737] Definition: Any process that modulates the frequency, rate or extent of (R)-mevalonic acid biosynthetic process.